{
  "gene_symbol": "PGP",
  "gene_name": "Glycerol-3-phosphate phosphatase",
  "term_label": "Unknown biological process",
  "gene": "UniProtKB:A6NDG6",
  "term_id": "UNKNOWN:0002"
}